prostaglandin D2 receptor binding [GO:0031863] (molecular function) Definition: Binding to a prostaglandin D2 receptor. Also known as: prostanoid DP receptor binding, prostaglandin D2 receptor ligand Relationships: is_a prostanoid receptor binding [GO:0031862] Sources: GOC:mah, GOC:nln